response to DNA integrity checkpoint signaling [GO:0072402] (biological process) Sources: GOC:mtg_cell_cycle Definition: A process that occurs in response to signals generated as a result of DNA integrity checkpoint signaling. Relationships: is a type of GO:0072396 Regulation: regulated by regulation of response to DNA integrity checkpoint signaling [GO:1902151]; positively regulated by positive regulation of response to DNA integrity checkpoint signaling [GO:1902152] Also known as: DNA integrity checkpoint effector process, response to signal involved in DNA integrity checkpoint Subtypes: response to DNA damage checkpoint signaling [GO:0072423], response to DNA replication checkpoint signaling [GO:0072438], response to mitotic DNA integrity checkpoint signaling [GO:1990820]